cellular response to isoquinoline alkaloid [GO:0071317] (biological process) Subtypes: cellular response to morphine [GO:0071315], cellular response to dextromethorphan [GO:1904559], cellular response to codeine [GO:1905234] Relationships: is a type of response to isoquinoline alkaloid [GO:0014072]; is a type of cellular response to alkaloid [GO:0071312] Sources: GOC:mah Definition: Any process that results in a change in state or activity of a cell (in terms of movement, secretion, enzyme production, gene expression, etc.) as a result of an isoquinoline alkaloid stimulus. An isoquinoline alkaloid is any member of a group of compounds with the heterocyclic ring structure of benzo(c)pyridine which is a structure characteristic of the group of opium alkaloids.